multivesicular body HOPS complex [GO:1902502] (cellular component) Definition: Any HOPS complex that is part of a multivesicular body membrane. Also known as: multivesicular body membrane HOPS complex Relationships: is a type of HOPS complex [GO:0030897]; is part of GO:0032585 References: PMID:23645161 Sources: GOC:TermGenie